procollagen-lysine 5-dioxygenase activity [GO:0008475] (molecular function) Definition: Catalysis of the reaction: L-lysyl-[collagen] + 2-oxoglutarate + O2 = (5R)-5-hydroxy-L-lysyl-[collagen] + succinate + CO2. Sources: RHEA:16569 Also known as: lysine hydroxylase activity, lysine,2-oxoglutarate 5-dioxygenase activity, lysine-2-oxoglutarate dioxygenase activity, lysyl hydroxylase activity, collagen lysine hydroxylase activity, lysylprotocollagen dioxygenase activity, procollagen-L-lysine,2-oxoglutarate:oxygen oxidoreductase (5-hydroxylating), procollagen-lysine,2-oxoglutarate 5-dioxygenase activity, protocollagen lysine dioxygenase activity, protocollagen lysine hydroxylase activity, protocollagen lysyl hydroxylase activity Relationships: is a type of 2-oxoglutarate-dependent dioxygenase activity [GO:0016706]; is_a GO:0140096